{
  "term_label": "Unknown biological process",
  "gene": "UniProtKB:Q5TAP6",
  "gene_symbol": "UTP14C",
  "gene_name": "U3 small nucleolar RNA-associated protein 14 homolog C",
  "term_id": "UNKNOWN:0002"
}